{
  "gene_name": "Tumor protein p53-inducible nuclear protein 2",
  "term_id": "GO:0045893",
  "gene": "UniProtKB:Q8IXH6",
  "gene_symbol": "TP53INP2",
  "term_label": "positive regulation of DNA-templated transcription"
}